osmosensory signaling pathway [GO:0007231] (biological process) Definition: The series of molecular signals initiated in response to osmotic change. Subtypes: osmosensory signaling pathway via Sho1 osmosensor [GO:0007232], osmosensory signaling via phosphorelay pathway [GO:0007234] Relationships: is a type of intracellular signal transduction [GO:0035556]; is a type of cellular response to osmotic stress [GO:0071470] Sources: GOC:jl Also known as: osmolarity sensing, osmolarity sensing signaling pathway, osmolarity sensing signalling pathway, osmosensory signal transduction, osmosensory signalling pathway, signal transduction during osmotic stress